{
  "term_label": "Cul2-RING ubiquitin ligase complex",
  "gene_name": "PRAME family member 25",
  "gene_symbol": "PRAMEF25",
  "gene": "UniProtKB:A6NGN4",
  "term_id": "GO:0031462"
}